positive regulation of TORC1 signaling [GO:1904263] (biological process) References: PMID:25366275 Sources: GOC:TermGenie, GO_REF:0000058 Relationships: is_a GO:0032008; is a type of regulation of TORC1 signaling [GO:1903432]; positively regulates TORC1 signaling [GO:0038202] Also known as: positive regulation of TORC1 signal transduction, up regulation of TORC1 signal transduction, up regulation of TORC1 signaling, up-regulation of TORC1 signal transduction, up-regulation of TORC1 signaling, upregulation of TORC1 signal transduction, upregulation of TORC1 signaling, activation of TORC1 signal transduction, activation of TORC1 signaling Definition: Any process that activates or increases the frequency, rate or extent of TORC1 signaling.